MCM complex binding [GO:1904931] (molecular function) Definition: Binding to an MCM complex. Relationships: is_a protein-containing complex binding [GO:0044877] Also known as: mini-chromosome maintenance complex binding References: PMID:12604790 Sources: GOC:TermGenie